{
  "term_label": "Unknown biological process",
  "term_id": "UNKNOWN:0002",
  "gene_name": "T cell receptor beta joining 2-3",
  "gene": "UniProtKB:A0A0B4J200",
  "gene_symbol": "TRBJ2-3"
}